{
  "term_id": "GO:0006427",
  "term_label": "histidyl-tRNA aminoacylation",
  "gene_symbol": "HARS1",
  "gene": "UniProtKB:P12081",
  "gene_name": "Histidine--tRNA ligase, cytoplasmic"
}